{
  "gene_symbol": "ST8SIA4",
  "term_label": "N-glycan processing",
  "gene_name": "CMP-N-acetylneuraminate-poly-alpha-2,8-sialyltransferase",
  "gene": "UniProtKB:Q92187",
  "term_id": "GO:0006491"
}